{
  "gene_name": "Calcineurin-binding protein cabin-1",
  "gene_symbol": "CABIN1",
  "term_label": "nucleus",
  "term_id": "GO:0005634",
  "gene": "UniProtKB:Q9Y6J0"
}